{
  "gene_symbol": "SPAAR",
  "gene": "UniProtKB:A0A1B0GVQ0",
  "gene_name": "Small regulatory polypeptide of amino acid response",
  "term_label": "Unknown biological process",
  "term_id": "UNKNOWN:0002"
}